{
  "term_id": "GO:0003984",
  "gene_symbol": "ILVBL",
  "gene_name": "2-hydroxyacyl-CoA lyase 2",
  "gene": "UniProtKB:A1L0T0",
  "term_label": "acetolactate synthase activity"
}